maintenance of CRISPR repeat elements [GO:0043571] (biological process) Also known as: maintenance of clustered regularly interspaced short palindromic repeat elements, CRISPR element metabolic process, CRISPR element metabolism Relationships: is a type of maintenance of DNA repeat elements [GO:0043570] Definition: Any process involved in sustaining CRISPR repeat clusters, including capture of new spacer elements, expansion or contraction of clusters, propagation of the leader sequence and repeat clusters within a genome, transfer of repeat clusters and CRISPR-associated (cas) genes to new genomes, transcription of the CRISPR repeat arrays into RNA and processing, and interaction of CRISPR/cas loci with the host genome. CRISPR (clustered regularly interspaced short palindromic repeat) elements are a family of sequence elements containing multiple direct repeats of 24-48 bp with weak dyad symmetry which are separated by regularly sized nonrepetitive spacer sequences. References: PMID:16292354